{
  "term_label": "wybutosine biosynthetic process",
  "gene": "UniProtKB:Q53H54",
  "gene_symbol": "TRMT12",
  "gene_name": "tRNA wybutosine-synthesizing protein 2 homolog",
  "term_id": "GO:0031591"
}